{
  "gene": "UniProtKB:Q13835",
  "term_id": "GO:0005886",
  "gene_symbol": "PKP1",
  "gene_name": "Plakophilin-1",
  "term_label": "plasma membrane"
}